{
  "term_id": "UNKNOWN:0003",
  "gene": "UniProtKB:Q96IW7",
  "gene_symbol": "SEC22A",
  "term_label": "Unknown cellular component",
  "gene_name": "Vesicle-trafficking protein SEC22a"
}